cumulus cell differentiation [GO:0001549] (biological process) Regulation: regulated by regulation of cumulus cell differentiation [GO:0045592]; negatively regulated by negative regulation of cumulus cell differentiation [GO:0045593]; positively regulated by positive regulation of cumulus cell differentiation [GO:0045594] Relationships: is a type of developmental process involved in reproduction [GO:0003006]; is a type of GO:0060014; is part of antral ovarian follicle growth [GO:0001547]; is part of fused antrum stage [GO:0048165] References: PMID:30010832 Definition: The process in which a subpopulation of granulosa cells surrounding the oocyte acquires the specialized features of an ovarian cumulus cell. Also known as: ovarian cumulus cell differentiation